regulation of nuclear-transcribed mRNA poly(A) tail shortening [GO:0060211] (biological process) Definition: Any process that modulates the frequency, rate or extent of poly(A) tail shortening of a nuclear-transcribed mRNA. Poly(A) tail shortening is the decrease in length of the poly(A) tail of an mRNA from full length to an oligo(A) length. Relationships: is_a GO:0061013; RO_0002211 nuclear-transcribed mRNA poly(A) tail shortening [GO:0000289] Also known as: regulation of 3' to 5' mRNA deadenylation, regulation of mRNA deadenylation, regulation of nuclear mRNA poly(A) tail shortening Subtypes: negative regulation of nuclear-transcribed mRNA poly(A) tail shortening [GO:0060212], positive regulation of nuclear-transcribed mRNA poly(A) tail shortening [GO:0060213] Sources: GOC:dph, GOC:tb